{
  "term_label": "Unknown cellular component",
  "gene_name": "Carbohydrate sulfotransferase 10",
  "gene": "UniProtKB:O43529",
  "gene_symbol": "CHST10",
  "term_id": "UNKNOWN:0003"
}